{
  "gene_symbol": "LINC00472",
  "gene": "UniProtKB:Q9H8W2",
  "term_label": "Unknown biological process",
  "gene_name": "Putative uncharacterized protein encoded by LINC00472",
  "term_id": "UNKNOWN:0002"
}